CD8-positive, alpha-beta T cell activation [GO:0036037] (biological process) Relationships: is a type of GO:0046631 Definition: The change in morphology and behavior of a CD8-positive, alpha-beta T cell resulting from exposure to a mitogen, cytokine, chemokine, cellular ligand, or an antigen for which it is specific. Regulation: RO_0002211 by GO:2001185; negatively regulated by negative regulation of CD8-positive, alpha-beta T cell activation [GO:2001186]; positively regulated by positive regulation of CD8-positive, alpha-beta T cell activation [GO:2001187] Sources: CL:0000625, GOC:yaf Subtypes: GO:0035740, CD8-positive, alpha-beta T cell differentiation [GO:0043374]